{
  "gene_name": "Transmembrane protein 241",
  "gene_symbol": "TMEM241",
  "term_label": "GDP-mannose transmembrane transporter activity",
  "term_id": "GO:0005458",
  "gene": "UniProtKB:Q24JQ0"
}